specification of segmental identity, abdomen [GO:0007385] (BP) Sources: ISBN:0878932437 Definition: The specification of the characteristic structures of the abdominal segments following establishment of segment boundaries. Identity is considered to be the aggregate of characteristics by which a structure is recognized. Relationships: is a type of specification of segmental identity, trunk [GO:0035292]